2,6-dioxo-6-phenylhexa-3-enoate hydrolase activity [GO:0018774] (molecular function) Sources: RHEA:17161 Also known as: 2-hydroxy-6-oxo-6-phenylhexa-2,4-dienoate hydrolase activity, 2,6-dioxo-6-phenylhexa-3-enoate benzoylhydrolase activity, HOHPDA hydrolase activity Relationships: is a type of hydrolase activity, acting on acid carbon-carbon bonds, in ketonic substances [GO:0016823] Definition: Catalysis of the reaction: 2,6-dioxo-6-phenylhexa-3-enoate + H2O = 2-oxopent-4-enoate + benzoate + H+.